protein transport from ciliary membrane to plasma membrane [GO:1903445] (BP) Definition: The directed movement of protein from ciliary membrane to plasma membrane. Relationships: is a type of protein transport within lipid bilayer [GO:0032594]; is a type of establishment of protein localization to plasma membrane [GO:0061951]; is a type of protein localization to plasma membrane [GO:0072659] References: PMID:22139371 Sources: GOC:TermGenie, GOC:cilia, GOC:krc, GO_REF:0000078